peptidase regulator activity [GO:0061134] (molecular function) Subtypes: peptidase activator activity [GO:0016504], peptidase inhibitor activity [GO:0030414], endopeptidase regulator activity [GO:0061135] Relationships: is a type of enzyme regulator activity [GO:0030234]; has part GO:0002020; regulates peptidase activity [GO:0008233] Definition: Binds to and modulates the activity of a peptidase, any enzyme that catalyzes the hydrolysis peptide bonds. Sources: GOC:dph, GOC:tb